relaxation of muscle [GO:0090075] (biological process) Regulation: regulated by regulation of relaxation of muscle [GO:1901077]; negatively regulated by negative regulation of relaxation of muscle [GO:1901078]; positively regulated by positive regulation of relaxation of muscle [GO:1901079] Relationships: is a type of muscle system process [GO:0003012] References: PMID:19996365 Sources: GOC:BHF, GOC:rl Subtypes: GO:0044557, GO:0055119, relaxation of skeletal muscle [GO:0090076] Definition: A process in which the extent of muscle contraction is reduced. Muscle relaxation can involve a number of processes including the removal of calcium from the cytoplasm to the sarcoplasmic reticulum lumen through the action of Ca2+ ATPases. In some muscles, calcium-independent pathways also play a role in muscle relaxation by decreasing the phosphorylation state of myosin light chain.